{
  "term_label": "plasma membrane",
  "term_id": "GO:0005886",
  "gene_symbol": "FAP",
  "gene": "UniProtKB:Q12884",
  "gene_name": "Prolyl endopeptidase FAP"
}